{
  "gene_name": "Fascin-2",
  "gene": "UniProtKB:O14926",
  "gene_symbol": "FSCN2",
  "term_label": "cytoplasm",
  "term_id": "GO:0005737"
}